{
  "gene_symbol": "HTR5A",
  "gene": "UniProtKB:P47898",
  "term_id": "GO:0007268",
  "gene_name": "5-hydroxytryptamine receptor 5A",
  "term_label": "chemical synaptic transmission"
}